immune response-inhibiting signal transduction [GO:0002765] (BP) Definition: The cascade of processes by which a signal interacts with a receptor, causing a change in the level or activity of a second messenger or other downstream target, and ultimately leading to inhibition of an immune response. Sources: GOC:add, ISBN:0781735149 Relationships: is a type of immune response-regulating signaling pathway [GO:0002764] Subtypes: GO:0002766, immune response-inhibiting cell surface receptor signaling pathway [GO:0002767]